MutSalpha complex binding [GO:0032407] (molecular function) Definition: Binding to a MutSalpha mismatch repair complex. Sources: GOC:vk Relationships: is a type of mismatch repair complex binding [GO:0032404]